{
  "term_id": "UNKNOWN:0002",
  "gene_name": "Wings apart-like protein homolog",
  "term_label": "Unknown biological process",
  "gene": "UniProtKB:Q7Z5K2",
  "gene_symbol": "WAPL"
}